{
  "gene_name": "HLA class II histocompatibility antigen, DRB1 beta chain",
  "gene_symbol": "HLA-DRB1",
  "gene": "UniProtKB:P01911",
  "term_label": "MHC class II protein complex binding",
  "term_id": "GO:0023026"
}